{
  "term_label": "nuclear-transcribed mRNA poly(A) tail shortening",
  "term_id": "GO:0000289",
  "gene": "UniProtKB:P26651",
  "gene_symbol": "ZFP36",
  "gene_name": "mRNA decay activator protein ZFP36"
}